protein localization to vacuolar membrane [GO:1903778] (biological process) References: PMID:25378562 Sources: GOC:TermGenie, GO_REF:0000087 Relationships: is_a protein localization to membrane [GO:0072657]; is a type of protein localization to vacuole [GO:0072665] Definition: A process in which a protein is transported to, or maintained in, a location within a vacuolar membrane. Subtypes: protein targeting to vacuolar membrane [GO:0044395] Also known as: protein localisation in vacuolar membrane, protein localisation to vacuolar membrane, protein localization in vacuolar membrane